positive regulation of estradiol secretion [GO:2000866] (biological process) Sources: GOC:sl Definition: Any process that activates or increases the frequency, rate or extent of estradiol secretion. Also known as: positive regulation of oestradiol secretion Relationships: is a type of positive regulation of steroid hormone secretion [GO:2000833]; is a type of regulation of estradiol secretion [GO:2000864]; positively regulates estradiol secretion [GO:0035938]